positive regulation of basement membrane assembly involved in embryonic body morphogenesis [GO:1904261] (biological process) Also known as: up regulation of basement membrane assembly involved in embryonic body morphogenesis, up-regulation of basement membrane assembly involved in embryonic body morphogenesis, upregulation of basement membrane assembly involved in embryonic body morphogenesis, activation of basement membrane assembly involved in embryonic body morphogenesis Definition: Any process that activates or increases the frequency, rate or extent of basement membrane assembly involved in embryonic body morphogenesis. Relationships: is a type of positive regulation of developmental process [GO:0051094]; is a type of GO:1901203; is a type of regulation of basement membrane assembly involved in embryonic body morphogenesis [GO:1904259]; positively regulates basement membrane assembly involved in embryonic body morphogenesis [GO:2001197] References: PMID:23940118 Sources: GOC:TermGenie, GOC:als, GO_REF:0000058